{
  "term_label": "protein folding",
  "gene": "UniProtKB:Q9H819",
  "gene_symbol": "DNAJC18",
  "gene_name": "DnaJ homolog subfamily C member 18",
  "term_id": "GO:0006457"
}